tyrosine decarboxylase activity [GO:0004837] (MF) Relationships: is_a GO:0016831 Also known as: L-(-)-tyrosine apodecarboxylase activity, L-tyrosine carboxy-lyase (tyramine-forming), L-tyrosine carboxy-lyase activity, L-tyrosine decarboxylase activity Definition: Catalysis of the reaction: L-tyrosine = tyramine + CO2. Sources: EC:4.1.1.25